{
  "term_id": "GO:0004984",
  "gene": "UniProtKB:Q8NGG8",
  "term_label": "olfactory receptor activity",
  "gene_symbol": "OR8B3",
  "gene_name": "Olfactory receptor 8B3"
}